{
  "term_label": "cytoplasm",
  "gene": "UniProtKB:Q14674",
  "term_id": "GO:0005737",
  "gene_symbol": "ESPL1",
  "gene_name": "Separin"
}